{
  "term_id": "UNKNOWN:0003",
  "term_label": "Unknown cellular component",
  "gene": "UniProtKB:Q9NS37",
  "gene_symbol": "CREBZF",
  "gene_name": "CREB_ATF bZIP transcription factor"
}